dATP diphosphatase activity [GO:0008828] (molecular function) Also known as: 2-hydroxy-(d)ATP pyrophosphatase activity, 2-hydroxy-(deoxy)adenosine-triphosphate pyrophosphatase activity, dATP pyrophosphohydrolase activity, 2-hydroxy-ATP pyrophosphatase activity, 2-hydroxy-adenosine triphosphate pyrophosphatase activity References: PMID:11139615 Sources: GOC:pde, RHEA:28334 Relationships: is a type of GO:0047429 Definition: Catalysis of the reaction: dATP + H2O = dAMP + H+ + diphosphate.